positive regulation of maltoheptaose transport [GO:1900308] (biological process) Relationships: is a type of GO:1900296; is a type of regulation of maltoheptaose transport [GO:1900306]; positively regulates GO:2001105 Sources: GOC:TermGenie, GOC:mengo_curators Definition: Any process that activates or increases the frequency, rate or extent of maltoheptaose transport. Also known as: up regulation of maltoheptaose transport, up-regulation of maltoheptaose transport, upregulation of maltoheptaose transport, activation of maltoheptaose transport